{
  "gene_symbol": "PCM1",
  "term_label": "non-motile cilium assembly",
  "gene_name": "Pericentriolar material 1 protein",
  "gene": "UniProtKB:Q15154",
  "term_id": "GO:1905515"
}